{
  "gene_symbol": "ZNF181",
  "gene": "UniProtKB:Q2M3W8",
  "term_label": "DNA-binding transcription factor activity, RNA polymerase II-specific",
  "gene_name": "Zinc finger protein 181",
  "term_id": "GO:0000981"
}